{
  "term_id": "GO:0048240",
  "term_label": "sperm capacitation",
  "gene_symbol": "ELSPBP1",
  "gene_name": "Epididymal sperm-binding protein 1",
  "gene": "UniProtKB:Q96BH3"
}